{
  "term_label": "vascular endothelial growth factor signaling pathway",
  "term_id": "GO:0038084",
  "gene_symbol": "VEGFA",
  "gene": "UniProtKB:P15692",
  "gene_name": "Vascular endothelial growth factor A, long form"
}